positive regulation of mitochondrial membrane potential [GO:0010918] (biological process) Definition: Any process that activates or increases the frequency, rate or extent of establishment or extent of a mitochondrial membrane potential, the electric potential existing across any mitochondrial membrane arising from charges in the membrane itself and from the charges present in the media on either side of the membrane. Also known as: elevation of mitochondrial membrane potential Sources: GOC:dph, GOC:tb Relationships: is a type of positive regulation of membrane potential [GO:0045838]; is a type of regulation of mitochondrial membrane potential [GO:0051881]